{
  "term_label": "Unknown molecular function",
  "gene": "UniProtKB:Q15061",
  "term_id": "UNKNOWN:0001",
  "gene_symbol": "WDR43",
  "gene_name": "WD repeat-containing protein 43"
}